{
  "gene": "UniProtKB:P04234",
  "term_label": "transmembrane signaling receptor activity",
  "term_id": "GO:0004888",
  "gene_symbol": "CD3D",
  "gene_name": "T-cell surface glycoprotein CD3 delta chain"
}